negative regulation of L-glutamine import across plasma membrane [GO:1901035] (biological process) Also known as: down-regulation of L-glutamine import, negative regulation of L-glutamine import, down regulation of L-glutamine import, down regulation of L-glutamine uptake, down-regulation of L-glutamine uptake, downregulation of L-glutamine import, downregulation of L-glutamine uptake, inhibition of L-glutamine uptake, negative regulation of L-glutamine uptake, inhibition of L-glutamine import Sources: GOC:TermGenie Definition: Any process that stops, prevents or reduces the frequency, rate or extent of L-glutamine import into a cell. Relationships: is a type of negative regulation of transmembrane transport [GO:0034763]; is a type of regulation of L-glutamine import across plasma membrane [GO:1901034]; is a type of negative regulation of glutamine transport [GO:2000486]; negatively regulates GO:1903803